{
  "term_id": "UNKNOWN:0001",
  "gene_name": "Transmembrane protein 14C",
  "gene": "UniProtKB:Q9P0S9",
  "term_label": "Unknown molecular function",
  "gene_symbol": "TMEM14C"
}